{
  "gene_name": "NADPH oxidase activator 1",
  "gene_symbol": "NOXA1",
  "term_id": "GO:0016176",
  "term_label": "superoxide-generating NADPH oxidase activator activity",
  "gene": "UniProtKB:Q86UR1"
}